{
  "term_id": "GO:0005102",
  "gene_name": "Protein cornichon homolog 4",
  "gene_symbol": "CNIH4",
  "gene": "UniProtKB:Q9P003",
  "term_label": "signaling receptor binding"
}